L-alanine biosynthetic process via ornithine [GO:0019273] (biological process) Also known as: L-alanine anabolism via ornithine, L-alanine formation via ornithine, L-alanine synthesis via ornithine Definition: The chemical reactions and pathways resulting in the formation of L-alanine, via the intermediate ornithine. Sources: GOC:go_curators Relationships: is a type of ornithine metabolic process [GO:0006591]; is a type of L-alanine biosynthetic process [GO:0042852]